{
  "gene_name": "5-azacytidine-induced protein 2",
  "term_label": "cytoplasm",
  "gene": "UniProtKB:Q9H6S1",
  "gene_symbol": "AZI2",
  "term_id": "GO:0005737"
}